negative regulation of neuron projection regeneration [GO:0070571] (biological process) Subtypes: GO:0048681 Sources: GOC:mah Also known as: growth cone collapse Relationships: is a type of negative regulation of neuron projection development [GO:0010977]; is a type of negative regulation of response to stimulus [GO:0048585]; is a type of GO:0051093; is a type of regulation of neuron projection regeneration [GO:0070570]; negatively regulates neuron projection regeneration [GO:0031102] Definition: Any process that stops, prevents, or reduces the frequency, rate or extent of neuron projection regeneration, the regrowth of neuronal processes such as axons or dendrites following their loss or damage.